{
  "term_label": "Unknown molecular function",
  "gene": "UniProtKB:A0A6Q8PGL7",
  "term_id": "UNKNOWN:0001",
  "gene_symbol": "A0A6Q8PGL7",
  "gene_name": "Uncharacterized protein"
}